{
  "term_id": "GO:0007218",
  "term_label": "neuropeptide signaling pathway",
  "gene_symbol": "NPFFR2",
  "gene_name": "Neuropeptide FF receptor 2",
  "gene": "UniProtKB:Q9Y5X5"
}